diacetylchitobiose catabolic process [GO:0052777] (biological process) Definition: The chemical reactions and pathways resulting in the breakdown of diacetylchitobiose into simpler products. Relationships: is_a diacetylchitobiose metabolic process [GO:0052778]; is a type of carbohydrate derivative catabolic process [GO:1901136] References: PMID:22797760 Also known as: diacetylchitobiose catabolism